{
  "term_id": "GO:0035368",
  "term_label": "selenocysteine insertion sequence binding",
  "gene_symbol": "SECISBP2",
  "gene_name": "Selenocysteine insertion sequence-binding protein 2",
  "gene": "UniProtKB:Q96T21"
}